{
  "gene": "UniProtKB:Q9NQS3",
  "gene_name": "Nectin-3",
  "gene_symbol": "NECTIN3",
  "term_label": "heterophilic cell-cell adhesion",
  "term_id": "GO:0007157"
}